{
  "term_label": "regulation of transcription by RNA polymerase II",
  "term_id": "GO:0006357",
  "gene_name": "Zinc finger protein 571",
  "gene_symbol": "ZNF571",
  "gene": "UniProtKB:Q7Z3V5"
}